{
  "gene_name": "Pro-interleukin-16",
  "gene_symbol": "IL16",
  "term_label": "CD4 receptor binding",
  "gene": "UniProtKB:Q14005",
  "term_id": "GO:0042609"
}